poly(A)-dependent snoRNA 3'-end processing [GO:0071051] (biological process) Relationships: is a type of sno(s)RNA 3'-end processing [GO:0031126] Also known as: polyadenylation-dependent snoRNA 3'-end processing, sno(s)RNA polyadenylation References: PMID:18951092 Sources: GOC:dgf, GOC:krc Definition: Any process involved in forming the mature 3' end of a snoRNA molecule linked to prior polyadenylation of the 3'-end of the precursor snoRNA.